{
  "gene": "UniProtKB:Q9UJU2",
  "term_id": "GO:1990907",
  "term_label": "beta-catenin-TCF complex",
  "gene_name": "Lymphoid enhancer-binding factor 1",
  "gene_symbol": "LEF1"
}